{
  "gene_symbol": "BAHD1",
  "term_id": "GO:0003682",
  "gene": "UniProtKB:Q8TBE0",
  "term_label": "chromatin binding",
  "gene_name": "Bromo adjacent homology domain-containing 1 protein"
}